{
  "gene": "UniProtKB:Q9UBP6",
  "gene_name": "tRNA (guanine-N(7)-)-methyltransferase",
  "gene_symbol": "METTL1",
  "term_label": "tRNA methylation",
  "term_id": "GO:0030488"
}